{
  "gene": "UniProtKB:P25054",
  "gene_name": "Adenomatous polyposis coli protein",
  "gene_symbol": "APC",
  "term_label": "negative regulation of microtubule depolymerization",
  "term_id": "GO:0007026"
}